pyruvate dehydrogenase (quinone) activity [GO:0052737] (molecular function) Relationships: is_a GO:0052738 Sources: EC:1.2.5.1 Definition: Catalysis of the reaction: a ubiquinone + H2O + pyruvate = a ubiquinol + acetate + CO2. Also known as: pyruvate dehydrogenase activity, pyruvic dehydrogenase activity, pyruvate:ubiquinone oxidoreductase activity, pyruvate:ubiquinone-8-oxidoreductase activity